{
  "gene_symbol": "NDUFS4",
  "term_id": "GO:0022904",
  "term_label": "respiratory electron transport chain",
  "gene": "UniProtKB:O43181",
  "gene_name": "NADH dehydrogenase [ubiquinone] iron-sulfur protein 4, mitochondrial"
}